{
  "term_id": "UNKNOWN:0002",
  "gene_symbol": "GPR141",
  "term_label": "Unknown biological process",
  "gene_name": "Probable G-protein coupled receptor 141",
  "gene": "UniProtKB:Q7Z602"
}